symbiont-mediated perturbation of host gene expression [GO:0039656] (BP) Subtypes: symbiont-mediated perturbation of host translation [GO:0019057], symbiont-mediated suppression of host mRNA processing [GO:0039524], symbiont-mediated degradation of host mRNA [GO:0039595], symbiont-mediated suppression of host transcription initiation from RNA polymerase II promoter [GO:0039602], symbiont-mediated suppression of host translation initiation [GO:0039606], GO:0039657, GO:0046773, symbiont-mediated perturbation of host transcription [GO:0052026], symbiont-mediated suppression of host translation elongation [GO:0141155] Relationships: is a type of symbiont-mediated perturbation of host cellular process [GO:0044068] Also known as: modulation by virus of host gene expression, regulation by virus of host gene expression Sources: GOC:bf Definition: A process in which a symbiont alters or subverts the normal execution of host gene expression. Gene expression is the process in which a gene's coding sequence is converted into a mature gene product or products (proteins or RNA). This includes the production of an RNA transcript as well as any processing to produce a mature RNA product or an mRNA (for protein-coding genes) and the translation of that mRNA into protein. Some protein processing events may be included when they are required to form an active form of a product from an inactive precursor form. The host is defined as the larger of the organisms involved in a symbiotic interaction.